{
  "gene_symbol": "FER1L6",
  "term_id": "UNKNOWN:0003",
  "gene_name": "Fer-1-like protein 6",
  "term_label": "Unknown cellular component",
  "gene": "UniProtKB:Q2WGJ9"
}